{
  "term_id": "GO:0016251",
  "gene_symbol": "GTF2B",
  "gene_name": "Transcription initiation factor IIB",
  "term_label": "RNA polymerase II general transcription initiation factor activity",
  "gene": "UniProtKB:Q00403"
}